{
  "gene_name": "Developmentally-regulated GTP-binding protein 2",
  "gene": "UniProtKB:P55039",
  "term_id": "GO:0005525",
  "term_label": "GTP binding",
  "gene_symbol": "DRG2"
}